{
  "gene_name": "TRAF-interacting protein with FHA domain-containing protein A",
  "term_id": "GO:0005737",
  "gene": "UniProtKB:Q96CG3",
  "gene_symbol": "TIFA",
  "term_label": "cytoplasm"
}